{
  "term_id": "GO:0048255",
  "gene_name": "Terminal nucleotidyltransferase 5A",
  "term_label": "mRNA stabilization",
  "gene": "UniProtKB:Q96IP4",
  "gene_symbol": "TENT5A"
}